{
  "term_id": "GO:0042761",
  "term_label": "very long-chain fatty acid biosynthetic process",
  "gene_name": "Very-long-chain (3R)-3-hydroxyacyl-CoA dehydratase 2",
  "gene_symbol": "HACD2",
  "gene": "UniProtKB:Q6Y1H2"
}